{
  "gene_name": "Insulin-like growth factor 2 mRNA-binding protein 3",
  "term_id": "GO:0005829",
  "term_label": "cytosol",
  "gene": "UniProtKB:O00425",
  "gene_symbol": "IGF2BP3"
}